{
  "gene_name": "Mitochondrial proton_calcium exchanger protein",
  "term_label": "mitochondrion organization",
  "term_id": "GO:0007005",
  "gene": "UniProtKB:O95202",
  "gene_symbol": "LETM1"
}